{
  "gene_name": "Limbic system-associated membrane protein",
  "term_label": "heterophilic cell-cell adhesion",
  "gene": "UniProtKB:Q13449",
  "gene_symbol": "LSAMP",
  "term_id": "GO:0007157"
}